{
  "term_label": "cytoplasm",
  "gene_name": "Adenylate kinase isoenzyme 5",
  "gene": "UniProtKB:Q9Y6K8",
  "term_id": "GO:0005737",
  "gene_symbol": "AK5"
}